{
  "term_id": "UNKNOWN:0002",
  "gene": "UniProtKB:Q9Y2B9",
  "term_label": "Unknown biological process",
  "gene_name": "cAMP-dependent protein kinase inhibitor gamma",
  "gene_symbol": "PKIG"
}